{
  "gene_symbol": "FUCA1",
  "gene": "UniProtKB:P04066",
  "term_label": "alpha-L-fucosidase activity",
  "term_id": "GO:0004560",
  "gene_name": "Tissue alpha-L-fucosidase"
}